3-hydroxypropionate dehydrogenase (NADP+) activity [GO:0035527] (molecular function) Definition: Catalysis of the reaction: 3-hydroxypropanoate + NADP+ = 3-oxopropanoate + H+ + NADPH. Sources: RHEA:26438 Also known as: 3-hydroxypropanoate dehydrogenase (NADP+) activity, 3-hydroxypropanoate:NADP+ oxidoreductase, 3-hydroxypropionate:NADP+ oxidoreductase Relationships: is a type of oxidoreductase activity, acting on the CH-OH group of donors, NAD or NADP as acceptor [GO:0016616]